{
  "term_id": "GO:0005125",
  "term_label": "cytokine activity",
  "gene_symbol": "WNT5A",
  "gene_name": "Protein Wnt-5a",
  "gene": "UniProtKB:P41221"
}